{
  "term_label": "cell surface receptor protein tyrosine kinase signaling pathway",
  "gene_name": "Embryonal Fyn-associated substrate",
  "gene": "UniProtKB:O43281",
  "gene_symbol": "EFS",
  "term_id": "GO:0007169"
}